{
  "gene_symbol": "FXN",
  "term_id": "GO:0005739",
  "gene_name": "Frataxin, mitochondrial",
  "gene": "UniProtKB:Q16595",
  "term_label": "mitochondrion"
}